{
  "gene_name": "Reticulon-2",
  "term_label": "postsynaptic density",
  "term_id": "GO:0014069",
  "gene_symbol": "RTN2",
  "gene": "UniProtKB:O75298"
}